{
  "gene_symbol": "ZMYM6",
  "term_id": "UNKNOWN:0001",
  "gene_name": "Zinc finger MYM-type protein 6",
  "gene": "UniProtKB:O95789",
  "term_label": "Unknown molecular function"
}